U2-type spliceosomal complex [GO:0005684] (cellular component) Definition: Any spliceosomal complex that forms during the splicing of a messenger RNA primary transcript to excise an intron that has canonical consensus sequences near the 5' and 3' ends. Note: A U2-type complex refers to any of the snRNP-based complexes that form during splicing that uses U2 (as opposed to U12). There are complexes that form during U2-splicing that don't necessarily contain the U2 snRNP. Relationships: is a type of spliceosomal complex [GO:0005681] References: PMID:11343900 Sources: GOC:krc, GOC:mah Also known as: major (U2-type) spliceosomal complex, major spliceosomal complex, GT-AG spliceosome Subtypes: commitment complex [GO:0000243], U2-type prespliceosome [GO:0071004], U2-type precatalytic spliceosome [GO:0071005], U2-type catalytic step 1 spliceosome [GO:0071006], GO:0071007, U2-type post-mRNA release spliceosomal complex [GO:0071008], U2-type post-spliceosomal complex [GO:0071021]